{
  "term_id": "GO:0043539",
  "gene_name": "STE20-related kinase adapter protein alpha",
  "gene": "UniProtKB:Q7RTN6",
  "term_label": "protein serine/threonine kinase activator activity",
  "gene_symbol": "STRADA"
}